{
  "gene_symbol": "SAAL1",
  "gene": "UniProtKB:Q96ER3",
  "gene_name": "Protein SAAL1",
  "term_id": "GO:0005654",
  "term_label": "nucleoplasm"
}